negative regulation of octadecene biosynthetic process [GO:1900915] (biological process) Definition: Any process that stops, prevents or reduces the frequency, rate or extent of octadecene biosynthetic process. Also known as: down regulation of octadecene biosynthetic process, down-regulation of octadecene biosynthetic process, downregulation of octadecene biosynthetic process, inhibition of 1-octadecene biosynthetic process, inhibition of octadecene anabolism, inhibition of octadecene biosynthesis, inhibition of octadecene biosynthetic process, inhibition of octadecene formation, inhibition of octadecene synthesis, down regulation of 1-octadecene biosynthetic process, down regulation of octadecene anabolism, down regulation of octadecene biosynthesis, down regulation of octadecene formation, down regulation of octadecene synthesis, down-regulation of 1-octadecene biosynthetic process, down-regulation of octadecene anabolism, down-regulation of octadecene biosynthesis, down-regulation of octadecene formation, down-regulation of octadecene synthesis, downregulation of 1-octadecene biosynthetic process, downregulation of octadecene anabolism, downregulation of octadecene biosynthesis, downregulation of octadecene formation, downregulation of octadecene synthesis, negative regulation of 1-octadecene biosynthetic process, negative regulation of octadecene anabolism, negative regulation of octadecene biosynthesis, negative regulation of octadecene formation, negative regulation of octadecene synthesis Sources: GOC:TermGenie, GOC:mengo_curators Relationships: is a type of negative regulation of olefin biosynthetic process [GO:1900912]; is a type of regulation of octadecene biosynthetic process [GO:1900914]; RO_0002212 octadecene biosynthetic process [GO:1900682]